{
  "gene_name": "Putative uncharacterized protein FLJ45355",
  "term_id": "UNKNOWN:0001",
  "gene": "UniProtKB:Q6ZSN1",
  "gene_symbol": "Q6ZSN1",
  "term_label": "Unknown molecular function"
}